{
  "gene_symbol": "HTR3C",
  "gene_name": "5-hydroxytryptamine receptor 3C",
  "term_label": "chemical synaptic transmission",
  "gene": "UniProtKB:Q8WXA8",
  "term_id": "GO:0007268"
}